{
  "gene_name": "Phosphoacetylglucosamine mutase",
  "gene_symbol": "PGM3",
  "term_label": "Unknown cellular component",
  "term_id": "UNKNOWN:0003",
  "gene": "UniProtKB:O95394"
}